regulation of centriole replication [GO:0046599] (biological process) Definition: Any process that modulates the frequency, rate or extent of the formation of a daughter centriole of an existing centriole. Subtypes: negative regulation of centriole replication [GO:0046600], positive regulation of centriole replication [GO:0046601] Sources: GOC:ai Relationships: is a type of regulation of centrosome duplication [GO:0010824]; is a type of regulation of organelle assembly [GO:1902115]; RO_0002211 centriole replication [GO:0007099]